{
  "gene_name": "Olfactory receptor 5M1",
  "term_label": "sensory perception of smell",
  "gene": "UniProtKB:Q8NGP8",
  "gene_symbol": "OR5M1",
  "term_id": "GO:0007608"
}